cholangiocyte apoptotic process [GO:1902488] (biological process) Also known as: epithelial cell of bile duct apoptotic process, cholangiocyte apoptosis, epithelial cell of bile duct apoptosis Definition: Any apoptotic process in a cholangiocyte. Regulation: regulated by regulation of cholangiocyte apoptotic process [GO:1904192]; RO_0002212 by negative regulation of cholangiocyte apoptotic process [GO:1904193]; positively regulated by GO:1904194 References: PMID:22961800 Sources: GOC:TermGenie Relationships: is a type of GO:1904019